{
  "term_id": "GO:0005737",
  "gene_symbol": "TRIM23",
  "term_label": "cytoplasm",
  "gene": "UniProtKB:P36406",
  "gene_name": "E3 ubiquitin-protein ligase TRIM23"
}